{
  "gene_name": "Myosin-14",
  "term_id": "GO:0032982",
  "gene_symbol": "MYH14",
  "gene": "UniProtKB:Q7Z406",
  "term_label": "myosin filament"
}